{
  "gene_symbol": "NARF",
  "term_id": "GO:0005638",
  "gene_name": "Nuclear prelamin A recognition factor",
  "gene": "UniProtKB:Q9UHQ1",
  "term_label": "lamin filament"
}